{
  "term_label": "intermediate filament organization",
  "gene_symbol": "KRT78",
  "gene_name": "Keratin, type II cytoskeletal 78",
  "gene": "UniProtKB:Q8N1N4",
  "term_id": "GO:0045109"
}